{
  "gene_name": "U4_U6.U5 tri-snRNP-associated protein 1",
  "term_id": "GO:0045292",
  "gene_symbol": "SART1",
  "term_label": "mRNA cis splicing, via spliceosome",
  "gene": "UniProtKB:O43290"
}